lipid phosphatase activity [GO:0042577] (molecular function) Sources: GOC:jl Relationships: is a type of phosphatase activity [GO:0016791] Subtypes: phosphatidate phosphatase activity [GO:0008195], sphingosine-1-phosphate phosphatase activity [GO:0042392], ceramide-1-phosphate phosphatase activity [GO:0106235] Definition: Catalysis of the reaction: a phospholipid + H2O = a lipid + phosphate.